{
  "gene_name": "p53 apoptosis effector related to PMP-22",
  "gene_symbol": "PERP",
  "gene": "UniProtKB:Q96FX8",
  "term_label": "Unknown molecular function",
  "term_id": "UNKNOWN:0001"
}